{
  "term_id": "GO:0045840",
  "gene_name": "Proepiregulin",
  "term_label": "positive regulation of mitotic nuclear division",
  "gene": "UniProtKB:O14944",
  "gene_symbol": "EREG"
}